{
  "term_label": "RNA polymerase II cis-regulatory region sequence-specific DNA binding",
  "term_id": "GO:0000978",
  "gene_name": "Zinc finger protein 485",
  "gene_symbol": "ZNF485",
  "gene": "UniProtKB:Q8NCK3"
}